{
  "gene": "UniProtKB:P53350",
  "term_id": "GO:0005737",
  "gene_symbol": "PLK1",
  "gene_name": "Serine_threonine-protein kinase PLK1",
  "term_label": "cytoplasm"
}